multicellular organismal response to stress [GO:0033555] (biological process) Definition: Any process that results in a change in state or activity of a multicellular organism (in terms of movement, secretion, enzyme production, gene expression, etc.) as a result of a stimulus indicating the organism is under stress. The stress is usually, but not necessarily, exogenous (e.g. temperature, humidity, ionizing radiation). Relationships: is a type of GO:0006950; is a type of GO:0032501 Sources: GOC:mah Subtypes: GO:0042596, response to pain [GO:0048265], general adaptation syndrome [GO:0051866]